{
  "term_label": "pyrimidine nucleobase biosynthetic process",
  "gene": "UniProtKB:P11172",
  "gene_symbol": "UMPS",
  "term_id": "GO:0019856",
  "gene_name": "Uridine 5'-monophosphate synthase"
}